negative regulation of binding [GO:0051100] (biological process) Sources: GOC:ai Subtypes: GO:0032091, GO:0035562, GO:0043392, GO:1900131 Also known as: down regulation of binding, down-regulation of binding, downregulation of binding, inhibition of binding Definition: Any process that stops or reduces the rate or extent of binding, the selective interaction of a molecule with one or more specific sites on another molecule. Relationships: is a type of negative regulation of molecular function [GO:0044092]; is_a regulation of binding [GO:0051098]; negatively regulates binding [GO:0005488]